methyl/ethyl malonyl-CoA decarboxylase activity [GO:0004492] (molecular function) Definition: Catalysis of the reaction: (S)-methylmalonyl-CoA + H+ = CO2 + propanoyl-CoA or (2S)-ethylmalonyl-CoA + H+ = butanoyl-CoA + CO2. Also known as: (S)-2-methyl-3-oxopropanoyl-CoA carboxy-lyase activity, (S)-methylmalonyl-CoA carboxy-lyase (propanoyl-CoA-forming), (S)-methylmalonyl-CoA carboxy-lyase activity, ethylmalonyl-CoA decarboxylase activity, methylmalonyl-coenzyme A decarboxylase activity Relationships: is a type of carboxy-lyase activity [GO:0016831] References: PMID:22016388